{
  "gene": "UniProtKB:Q5W0Q7",
  "gene_symbol": "USPL1",
  "term_label": "SUMO binding",
  "term_id": "GO:0032183",
  "gene_name": "SUMO-specific isopeptidase USPL1"
}